{
  "gene_symbol": "IGLJ1",
  "gene_name": "Immunoglobulin lambda joining 1",
  "gene": "UniProtKB:A0A0A0MT76",
  "term_id": "UNKNOWN:0001",
  "term_label": "Unknown molecular function"
}